{
  "gene_symbol": "CMKLR2",
  "gene_name": "Chemerin-like receptor 2",
  "gene": "UniProtKB:P46091",
  "term_label": "neuropeptide signaling pathway",
  "term_id": "GO:0007218"
}